{
  "term_label": "extracellular space",
  "gene": "UniProtKB:O00622",
  "gene_name": "CCN family member 1",
  "term_id": "GO:0005615",
  "gene_symbol": "CCN1"
}